methotrexate transmembrane transporter activity [GO:0015350] (molecular function) Definition: Enables the transfer of methotrexate, 4-amino-10-methylformic acid from one side of a membrane to the other. Methotrexate is a folic acid analogue and a potent competitive inhibitor of dihydrofolate reductase. Sources: GOC:ai Also known as: methotrexate transporter activity Relationships: is a type of GO:0005310; is a type of amide transmembrane transporter activity [GO:0042887]; is a type of xenobiotic transmembrane transporter activity [GO:0042910]; is part of methotrexate transport [GO:0051958]